{
  "term_label": "cytosol",
  "term_id": "GO:0005829",
  "gene": "UniProtKB:Q9HCE1",
  "gene_name": "Helicase MOV-10",
  "gene_symbol": "MOV10"
}